{
  "gene_symbol": "DCDC2",
  "term_id": "GO:0060091",
  "gene_name": "Doublecortin domain-containing protein 2",
  "gene": "UniProtKB:Q9UHG0",
  "term_label": "kinocilium"
}